regulation of collagen fibril organization [GO:1904026] (biological process) Also known as: regulation of collagen fibril organisation, regulation of fibrillar collagen organization, regulation of collagen fibrillogenesis Relationships: is a type of regulation of extracellular matrix organization [GO:1903053]; regulates collagen fibril organization [GO:0030199] Subtypes: negative regulation of collagen fibril organization [GO:1904027], positive regulation of collagen fibril organization [GO:1904028] Definition: Any process that modulates the frequency, rate or extent of collagen fibril organization. References: PMID:25451920 Sources: GOC:TermGenie, GO_REF:0000058